acylglycerol biosynthetic process [GO:0046463] (biological process) Relationships: is a type of acylglycerol metabolic process [GO:0006639]; is a type of glycerolipid biosynthetic process [GO:0045017]; is a type of GO:0046460 Also known as: acylglycerol anabolism, acylglycerol biosynthesis, acylglycerol formation, acylglycerol synthesis Definition: The chemical reactions and pathways resulting in the formation of acylglycerol, any mono-, di- or triester of glycerol with (one or more) fatty acids. Subtypes: monoacylglycerol biosynthetic process [GO:0006640], diacylglycerol biosynthetic process [GO:0006651], triglyceride biosynthetic process [GO:0019432] Sources: GOC:ai